{
  "term_label": "DNA-binding transcription factor activity, RNA polymerase II-specific",
  "gene_symbol": "ZKSCAN3",
  "gene_name": "Zinc finger protein with KRAB and SCAN domains 3",
  "term_id": "GO:0000981",
  "gene": "UniProtKB:Q9BRR0"
}